{
  "gene": "UniProtKB:Q9UII6",
  "gene_symbol": "DUSP13B",
  "term_id": "GO:0043409",
  "gene_name": "Dual specificity protein phosphatase 13 isoform B",
  "term_label": "negative regulation of MAPK cascade"
}